{
  "term_id": "GO:0001525",
  "gene": "UniProtKB:P50895",
  "gene_symbol": "BCAM",
  "term_label": "angiogenesis",
  "gene_name": "Basal cell adhesion molecule"
}